{
  "term_label": "NuA4 histone acetyltransferase complex",
  "gene_symbol": "EPC1",
  "term_id": "GO:0035267",
  "gene": "UniProtKB:Q9H2F5",
  "gene_name": "Enhancer of polycomb homolog 1"
}